{
  "term_label": "Wnt-protein binding",
  "gene_name": "Frizzled-3",
  "gene": "UniProtKB:Q9NPG1",
  "term_id": "GO:0017147",
  "gene_symbol": "FZD3"
}